{
  "term_id": "UNKNOWN:0001",
  "gene_name": "Endogenous retrovirus group K member 16 Rec protein",
  "gene": "UniProtKB:P61578",
  "term_label": "Unknown molecular function",
  "gene_symbol": "ERVK-16"
}